{
  "gene_symbol": "RRP9",
  "gene": "UniProtKB:O43818",
  "gene_name": "U3 small nucleolar RNA-interacting protein 2",
  "term_label": "small-subunit processome",
  "term_id": "GO:0032040"
}